{
  "term_label": "Unknown molecular function",
  "term_id": "UNKNOWN:0001",
  "gene_symbol": "NSL1",
  "gene": "UniProtKB:Q96IY1",
  "gene_name": "Kinetochore-associated protein NSL1 homolog"
}